acetoacetyl-CoA reductase activity [GO:0018454] (molecular function) Also known as: beta-ketoacyl-CoA reductase, (R)-3-hydroxyacyl-CoA dehydrogenase activity, (R)-3-hydroxyacyl-CoA:NADP+ oxidoreductase activity, D(-)-beta-hydroxybutyryl CoA-NADP oxidoreductase activity, D-3-hydroxyacyl-CoA reductase activity, NADP-linked acetoacetyl CoA reductase activity, NADPH:acetoacetyl-CoA reductase activity, acetoacetyl coenzyme A reductase activity, hydroxyacyl coenzyme-A dehydrogenase activity, short chain beta-ketoacetyl(acetoacetyl)-CoA reductase activity Relationships: is a type of oxidoreductase activity, acting on the CH-OH group of donors, NAD or NADP as acceptor [GO:0016616] Definition: Catalysis of the reaction: (R)-3-hydroxyacyl-CoA + NADP+ = 3-oxoacyl-CoA + NADPH + H+. Sources: EC:1.1.1.36